{
  "term_label": "plasma membrane",
  "gene_name": "Monocarboxylate transporter 6",
  "gene": "UniProtKB:O15375",
  "gene_symbol": "SLC16A5",
  "term_id": "GO:0005886"
}